{
  "gene_name": "Alpha-crystallin B chain",
  "term_id": "GO:0005737",
  "gene": "UniProtKB:P02511",
  "term_label": "cytoplasm",
  "gene_symbol": "CRYAB"
}